{
  "gene_name": "ALX homeobox protein 1",
  "gene": "UniProtKB:Q15699",
  "gene_symbol": "ALX1",
  "term_id": "GO:0048704",
  "term_label": "embryonic skeletal system morphogenesis"
}